cephamycin C catabolic process [GO:1901117] (biological process) Also known as: cephamycin C breakdown, cephamycin C catabolism, cephamycin C degradation Definition: The chemical reactions and pathways resulting in the breakdown of cephamycin C. Relationships: is a type of beta-lactam antibiotic catabolic process [GO:0030655]; is a type of sulfur compound catabolic process [GO:0044273] Sources: GOC:TermGenie, GOC:yaf, UniPathway:UPA00183